{
  "gene": "UniProtKB:P0DQW1",
  "gene_symbol": "SMIM46",
  "gene_name": "Small integral membrane protein 46",
  "term_label": "Unknown molecular function",
  "term_id": "UNKNOWN:0001"
}